{
  "gene_symbol": "GCK",
  "gene": "UniProtKB:P35557",
  "term_id": "GO:0050796",
  "gene_name": "Hexokinase-4",
  "term_label": "regulation of insulin secretion"
}